inclusion body assembly [GO:0070841] (biological process) Relationships: is a type of cellular component assembly [GO:0022607] Subtypes: aggresome assembly [GO:0070842], Lewy body formation [GO:0140121], neurofibrillary tangle assembly [GO:1902988] Sources: GOC:BHF, GOC:mah Regulation: RO_0002211 by regulation of inclusion body assembly [GO:0090083]; negatively regulated by negative regulation of inclusion body assembly [GO:0090084]; positively regulated by GO:0090261 Definition: The aggregation, arrangement and bonding together of a set of components to form an inclusion body.